{
  "gene": "UniProtKB:P61619",
  "gene_symbol": "SEC61A1",
  "gene_name": "Protein transport protein Sec61 subunit alpha isoform 1",
  "term_id": "GO:0008320",
  "term_label": "protein transmembrane transporter activity"
}